{
  "gene_name": "Exocyst complex component 4",
  "term_id": "GO:0032584",
  "gene": "UniProtKB:Q96A65",
  "gene_symbol": "EXOC4",
  "term_label": "growth cone membrane"
}